N-acetylglucosamine catabolic process [GO:0006046] (biological process) Definition: The chemical reactions and pathways resulting in the breakdown of N-acetylglucosamine. The D isomer is a common structural unit of glycoproteins in plants, bacteria and animals; it is often the terminal sugar of an oligosaccharide group of a glycoprotein. Sources: ISBN:0198506732 Also known as: N-acetylglucosamine breakdown, N-acetylglucosamine catabolism, N-acetylglucosamine degradation Relationships: is_a N-acetylglucosamine metabolic process [GO:0006044]; is a type of GO:1901072